{
  "term_label": "alpha-1,4-glucosidase activity",
  "gene_symbol": "GAA",
  "gene": "UniProtKB:P10253",
  "gene_name": "Lysosomal alpha-glucosidase",
  "term_id": "GO:0004558"
}